{
  "gene_symbol": "INMT",
  "term_id": "GO:0030748",
  "gene_name": "Indolethylamine N-methyltransferase",
  "term_label": "amine N-methyltransferase activity",
  "gene": "UniProtKB:O95050"
}